2-aminomuconate deaminase activity [GO:0050540] (molecular function) Definition: Catalysis of the reaction: 2-aminomuconate + H2O + H+ = (Z)-5-oxohex-2-enedioate + NH4. Sources: EC:3.5.99.5, RHEA:20996 Also known as: 2-aminomuconate aminohydrolase activity Relationships: is a type of deaminase activity [GO:0019239]